{
  "term_label": "Unknown molecular function",
  "gene": "UniProtKB:Q13287",
  "gene_name": "N-myc-interactor",
  "gene_symbol": "NMI",
  "term_id": "UNKNOWN:0001"
}